{
  "term_id": "GO:0003254",
  "gene": "UniProtKB:Q9Y3Q4",
  "gene_name": "Potassium_sodium hyperpolarization-activated cyclic nucleotide-gated channel 4",
  "term_label": "regulation of membrane depolarization",
  "gene_symbol": "HCN4"
}